{
  "gene": "UniProtKB:Q96RJ6",
  "term_id": "GO:0032502",
  "term_label": "developmental process",
  "gene_name": "Fer3-like protein",
  "gene_symbol": "FERD3L"
}